apical dendrite development [GO:0150022] (biological process) Relationships: is_a dendrite development [GO:0016358] References: PMID:22683681 Sources: GOC:aruk, GOC:bc Definition: The process whose specific outcome is the progression of an apical dendrite over time, from its formation to the mature structure.